{
  "term_label": "nerve growth factor receptor binding",
  "term_id": "GO:0005163",
  "gene_name": "Neurotrophin-3",
  "gene_symbol": "NTF3",
  "gene": "UniProtKB:P20783"
}